Kdo2-lipid IVA acyltransferase activity [GO:0008913] (molecular function) Also known as: (Kdo)2-lipid IVA lauroyltransferase, Kdo2-lipid IVA lauroyltransferase, alpha-Kdo-(2->4)-alpha-(2->6)-lipid IVA lauroyltransferase, lauroyl transferase activity, lauroyltransferase activity Definition: Catalysis of the reaction: a fatty acyl-[ACP] + an alpha-Kdo-(2->4)-alpha-Kdo-(2->6)-lipid IVA = an alpha-Kdo-(2->4)-alpha-Kdo-(2->6)-(acyl)-lipid IVA + holo-[ACP]. Relationships: is a type of GO:0016747 References: PMID:18656959 Sources: EC:2.3.1.241